{
  "gene_symbol": "IPP",
  "gene": "UniProtKB:Q9Y573",
  "term_label": "cytoplasm",
  "gene_name": "Actin-binding protein IPP",
  "term_id": "GO:0005737"
}